{
  "gene": "UniProtKB:P17643",
  "gene_name": "5,6-dihydroxyindole-2-carboxylic acid oxidase",
  "term_label": "melanosome",
  "gene_symbol": "TYRP1",
  "term_id": "GO:0042470"
}